{
  "gene": "UniProtKB:Q96A44",
  "term_id": "GO:0019005",
  "term_label": "SCF ubiquitin ligase complex",
  "gene_name": "SPRY domain-containing SOCS box protein 4",
  "gene_symbol": "SPSB4"
}